{
  "gene_symbol": "KRT39",
  "gene": "UniProtKB:Q6A163",
  "term_id": "GO:0030280",
  "term_label": "structural constituent of skin epidermis",
  "gene_name": "Keratin, type I cytoskeletal 39"
}